titin Z domain binding [GO:0070080] (molecular function) Sources: GOC:mah, InterPro:IPR015129 Definition: Binding to a titin Z protein domain, which recognizes and binds to the C-terminal calmodulin-like domain of alpha-actinin-2 (Act-EF34), adopts a helical structure, and binds in a groove formed by the two planes between the helix pairs of Act-EF34. Also known as: Z repeat domain binding Relationships: is_a GO:0019904